{
  "gene_name": "Putative zinc finger protein 355P",
  "term_label": "RNA polymerase II cis-regulatory region sequence-specific DNA binding",
  "term_id": "GO:0000978",
  "gene": "UniProtKB:Q9NSJ1",
  "gene_symbol": "ZNF355P"
}